female meiosis II [GO:0007147] (biological process) Definition: The cell cycle process in which the second meiotic division occurs in the female germline. Relationships: is a type of meiosis II [GO:0007135]; is_a female meiotic nuclear division [GO:0007143] Also known as: female meiosis II nuclear division Sources: GOC:mah